{
  "gene": "UniProtKB:Q9BY11",
  "term_label": "phospholipid binding",
  "gene_name": "Protein kinase C and casein kinase substrate in neurons protein 1",
  "term_id": "GO:0005543",
  "gene_symbol": "PACSIN1"
}